strictosidine synthase activity [GO:0016844] (molecular function) Also known as: 3-alpha(S)-strictosidine tryptamine-lyase (secologanin-forming), 3-alpha(S)-strictosidine tryptamine-lyase activity, STR activity, strictosidine synthetase activity Relationships: is a type of hydrolase activity, acting on carbon-nitrogen (but not peptide) bonds [GO:0016810] Definition: Catalysis of the reaction: 3alpha(S)-strictosidine + H2O = secologanin + tryptamine. Sources: RHEA:15013